{
  "gene": "UniProtKB:Q86Z20",
  "term_label": "Unknown molecular function",
  "term_id": "UNKNOWN:0001",
  "gene_symbol": "CCDC125",
  "gene_name": "Coiled-coil domain-containing protein 125"
}